{
  "term_id": "GO:0005737",
  "term_label": "cytoplasm",
  "gene": "UniProtKB:Q12774",
  "gene_name": "Rho guanine nucleotide exchange factor 5",
  "gene_symbol": "ARHGEF5"
}